{
  "term_id": "GO:0006629",
  "term_label": "lipid metabolic process",
  "gene_symbol": "FADS6",
  "gene": "UniProtKB:Q8N9I5",
  "gene_name": "Fatty acid desaturase 6"
}